{
  "gene": "UniProtKB:Q9H8T0",
  "gene_symbol": "AKTIP",
  "term_id": "GO:0070534",
  "term_label": "protein K63-linked ubiquitination",
  "gene_name": "AKT-interacting protein"
}